oxidoreductase activity, acting on the aldehyde or oxo group of donors, NAD or NADP as acceptor [GO:0016620] (molecular function) Subtypes: L-glutamate gamma-semialdehyde dehydrogenase activity [GO:0003842], N-acetyl-gamma-glutamyl-phosphate reductase activity [GO:0003942], 3-chloroallyl aldehyde dehydrogenase activity [GO:0004028], aldehyde dehydrogenase [NAD(P)+] activity [GO:0004030], aspartate-semialdehyde dehydrogenase activity [GO:0004073], glutamate-5-semialdehyde dehydrogenase activity [GO:0004350], methylmalonate-semialdehyde dehydrogenase (acylating, NAD) activity [GO:0004491], acetaldehyde dehydrogenase (acetylating) activity [GO:0008774], formate dehydrogenase (NAD+) activity [GO:0008863], GO:0008883, succinate-semialdehyde dehydrogenase [NAD(P)+] activity [GO:0009013], cinnamoyl-CoA reductase activity [GO:0016621], delta1-pyrroline-5-carboxylate synthetase activity [GO:0017084], GO:0018478, 5-carboxymethyl-2-hydroxymuconic-semialdehyde dehydrogenase activity [GO:0018480], 4-hydroxymuconic-semialdehyde dehydrogenase activity [GO:0018481], 4-formylbenzenesulfonate dehydrogenase activity [GO:0018482], 6-oxohexanoate dehydrogenase activity [GO:0018483], 2-oxobutyrate synthase activity [GO:0018491], malonate-semialdehyde dehydrogenase activity [GO:0033722], geranial dehydrogenase activity [GO:0034832], succinylglutamate-semialdehyde dehydrogenase activity [GO:0043824], N-acetyl-gamma-aminoadipyl-phosphate reductase activity [GO:0043870], GO:0043891, 2,5-dioxovalerate dehydrogenase (NAD+) activity [GO:0044104], aminomuconate-semialdehyde dehydrogenase activity [GO:0047102], 4-trimethylammoniobutyraldehyde dehydrogenase activity [GO:0047105], GO:0047110, (R)-dehydropantoate dehydrogenase activity [GO:0047509], 2,5-dioxovalerate dehydrogenase (NADP+) activity [GO:0047533], formate dehydrogenase (NADP+) activity [GO:0047899], glyoxylate dehydrogenase (acylating) activity [GO:0047968], erythrose-4-phosphate dehydrogenase activity [GO:0048001], long-chain-fatty-acyl-CoA reductase activity [GO:0050062], pyruvate dehydrogenase (NADP+) activity [GO:0050243], GO:0050607, vanillin dehydrogenase activity [GO:0050608], alpha-ketoester reductase (NADPH) activity [GO:0051269], 5-oxovalerate dehydrogenase activity [GO:0055043], alcohol-forming very long-chain fatty acyl-CoA reductase activity [GO:0080019], GO:0102810, alcohol-forming long-chain fatty acyl-CoA reductase activity [GO:0102965], sulfoacetaldehyde dehydrogenase activity [GO:0102984], glyceraldehyde-3-phosphate dehydrogenase [NAD(P)+] (non-phosphorylating) activity [GO:0120533] Relationships: is a type of oxidoreductase activity, acting on the aldehyde or oxo group of donors [GO:0016903] Sources: GOC:jl Definition: Catalysis of an oxidation-reduction (redox) reaction in which an aldehyde or ketone (oxo) group acts as a hydrogen or electron donor and reduces NAD or NADP.